{
  "term_label": "mRNA 3'-UTR AU-rich region binding",
  "gene_symbol": "ZFP36",
  "term_id": "GO:0035925",
  "gene": "UniProtKB:P26651",
  "gene_name": "mRNA decay activator protein ZFP36"
}